{
  "gene_symbol": "ZFP37",
  "term_id": "GO:0000981",
  "gene": "UniProtKB:Q9Y6Q3",
  "term_label": "DNA-binding transcription factor activity, RNA polymerase II-specific",
  "gene_name": "Zinc finger protein 37 homolog"
}